{
  "term_label": "semaphorin-plexin signaling pathway",
  "term_id": "GO:0071526",
  "gene_name": "Plexin-B2",
  "gene": "UniProtKB:O15031",
  "gene_symbol": "PLXNB2"
}